{
  "term_id": "GO:0005615",
  "gene_name": "Defensin beta 4A",
  "term_label": "extracellular space",
  "gene_symbol": "DEFB4B",
  "gene": "UniProtKB:O15263"
}